{
  "gene_symbol": "A0A7I2V4U8",
  "gene_name": "Uncharacterized protein",
  "term_id": "UNKNOWN:0003",
  "term_label": "Unknown cellular component",
  "gene": "UniProtKB:A0A7I2V4U8"
}